cytoneme [GO:0035230] (cellular component) Also known as: membrane nanotube Definition: A long, thin, polarized cell projection that contains actin and can extend for distances many times the diameter of the cell. Cytonemes represent extensions of cell cytoplasm and typically have a diameter of approximately 0.2um. Relationships: is a type of GO:0120025 References: PMID:10367889, PMID:10675901